{
  "gene": "UniProtKB:Q86X53",
  "term_label": "Unknown molecular function",
  "term_id": "UNKNOWN:0001",
  "gene_symbol": "ERICH1",
  "gene_name": "Glutamate-rich protein 1"
}